{
  "gene_symbol": "ARHGAP29",
  "gene_name": "Rho GTPase-activating protein 29",
  "term_id": "GO:0051058",
  "gene": "UniProtKB:Q52LW3",
  "term_label": "negative regulation of small GTPase mediated signal transduction"
}